{
  "gene_name": "Protein ARV1",
  "term_label": "Unknown molecular function",
  "term_id": "UNKNOWN:0001",
  "gene_symbol": "ARV1",
  "gene": "UniProtKB:Q9H2C2"
}